cerebellar Purkinje cell precursor proliferation [GO:0021925] (biological process) Definition: The multiplication or reproduction of neuroblasts that will give rise to Purkinje cells. A Purkinje cell is an inhibitory GABAergic neuron found in the cerebellar cortex that projects to the deep cerebellar nuclei and brain stem. References: PMID:15157725 Sources: GOC:cls, GOC:dgh, GOC:dph, GOC:jid, GO_REF:0000021 Relationships: is a type of GO:0021923